{
  "gene_name": "Ankyrin repeat domain-containing protein 13B",
  "gene": "UniProtKB:Q86YJ7",
  "gene_symbol": "ANKRD13B",
  "term_id": "GO:0140036",
  "term_label": "ubiquitin-modified protein reader activity"
}